{
  "term_label": "Unknown biological process",
  "gene_name": "Cytoplasmic phosphatidylinositol transfer protein 1",
  "term_id": "UNKNOWN:0002",
  "gene_symbol": "PITPNC1",
  "gene": "UniProtKB:Q9UKF7"
}